{
  "gene": "UniProtKB:O75437",
  "gene_symbol": "ZNF254",
  "term_label": "RNA polymerase II cis-regulatory region sequence-specific DNA binding",
  "term_id": "GO:0000978",
  "gene_name": "Zinc finger protein 254"
}